{
  "gene_symbol": "PTPRF",
  "term_label": "synaptic membrane adhesion",
  "gene": "UniProtKB:P10586",
  "gene_name": "Receptor-type tyrosine-protein phosphatase F",
  "term_id": "GO:0099560"
}